negative regulation of toll-like receptor 1 signaling pathway [GO:0034132] (biological process) Definition: Any process that stops, prevents, or reduces the frequency, rate, or extent of toll-like receptor 1 signaling pathway. Relationships: is a type of negative regulation of immune system process [GO:0002683]; is a type of GO:0009968; is a type of GO:0034131; negatively regulates toll-like receptor 1 signaling pathway [GO:0034130] References: PMID:16551253, PMID:17328678 Sources: GOC:add Also known as: negative regulation of TLR1 signaling pathway, negative regulation of toll-like receptor 1 signalling pathway